{
  "term_label": "frizzled binding",
  "gene": "UniProtKB:P54792",
  "gene_symbol": "DVL1P1",
  "term_id": "GO:0005109",
  "gene_name": "Putative segment polarity protein dishevelled homolog DVL1P1"
}